{
  "gene": "UniProtKB:Q9H082",
  "gene_name": "Ras-related protein Rab-33B",
  "term_id": "GO:0000045",
  "term_label": "autophagosome assembly",
  "gene_symbol": "RAB33B"
}